{
  "gene_symbol": "CDH5",
  "term_label": "catenin complex",
  "gene": "UniProtKB:P33151",
  "gene_name": "Cadherin-5",
  "term_id": "GO:0016342"
}